{
  "gene_symbol": "DUS3L",
  "term_id": "UNKNOWN:0002",
  "term_label": "Unknown biological process",
  "gene": "UniProtKB:Q96G46",
  "gene_name": "tRNA-dihydrouridine(47) synthase [NAD(P)(+)]-like"
}